{
  "term_label": "fatty acid binding",
  "gene_name": "Cellular retinoic acid-binding protein 1",
  "gene_symbol": "CRABP1",
  "term_id": "GO:0005504",
  "gene": "UniProtKB:P29762"
}